{
  "term_label": "polyamine transmembrane transporter activity",
  "term_id": "GO:0015203",
  "gene_symbol": "ATP13A4",
  "gene_name": "Probable cation-transporting ATPase 13A4",
  "gene": "UniProtKB:Q4VNC1"
}